phytochelatin-metal complex formation [GO:0090423] (biological process) Sources: GOC:tb Relationships: is a type of phytochelatin metabolic process [GO:0046937] Definition: A phytochelatin metabolic process in which a metal is incorporated with phytochelatin to form a complex. Also known as: LWM phytochelatin complex formation, low molecular weight phytochelatin complex formation